{
  "term_label": "cell-cell adhesion",
  "gene_symbol": "TLN1",
  "term_id": "GO:0098609",
  "gene": "UniProtKB:Q9Y490",
  "gene_name": "Talin-1"
}